{
  "gene_symbol": "GRIK1",
  "gene": "UniProtKB:P39086",
  "term_id": "GO:0042734",
  "term_label": "presynaptic membrane",
  "gene_name": "Glutamate receptor ionotropic, kainate 1"
}